negative regulation of zygospore formation [GO:0075300] (biological process) Relationships: is a type of negative regulation of sexual sporulation resulting in formation of a cellular spore [GO:0043942]; is_a regulation of zygospore formation [GO:0075298]; negatively regulates zygospore formation [GO:0034296] Definition: Any process that stops, prevents, or reduces the frequency, rate or extent of zygospore formation, a process in which a thick-walled spore of some algae and fungi is formed by union of two similar sexual cells, usually serves as a resting spore, and produces the sporophytic phase. Sources: GOC:pamgo_curators